{
  "term_label": "succinate-semialdehyde dehydrogenase (NAD+) activity",
  "gene_name": "Succinate-semialdehyde dehydrogenase, mitochondrial",
  "gene": "UniProtKB:P51649",
  "gene_symbol": "ALDH5A1",
  "term_id": "GO:0004777"
}